{
  "term_label": "plasma membrane",
  "gene_symbol": "NOS1",
  "gene_name": "Nitric oxide synthase 1",
  "gene": "UniProtKB:P29475",
  "term_id": "GO:0005886"
}